{
  "term_id": "GO:0070062",
  "gene_name": "G-protein coupled receptor family C group 5 member C",
  "gene": "UniProtKB:Q9NQ84",
  "term_label": "extracellular exosome",
  "gene_symbol": "GPRC5C"
}